regulation of sister chromatid segregation [GO:0033045] (BP) Definition: Any process that modulates the frequency, rate or extent of sister chromatid segregation. Relationships: is a type of regulation of chromosome organization [GO:0033044]; is a type of regulation of chromosome segregation [GO:0051983]; regulates sister chromatid segregation [GO:0000819] Sources: GOC:mah Subtypes: negative regulation of sister chromatid segregation [GO:0033046], GO:0033047, GO:0044784, GO:1902099